{
  "gene_symbol": "CPSF4",
  "gene": "UniProtKB:O95639",
  "gene_name": "Cleavage and polyadenylation specificity factor subunit 4",
  "term_id": "GO:0005847",
  "term_label": "mRNA cleavage and polyadenylation specificity factor complex"
}